{
  "term_id": "UNKNOWN:0002",
  "gene": "UniProtKB:O95157",
  "term_label": "Unknown biological process",
  "gene_symbol": "NXPH3",
  "gene_name": "Neurexophilin-3"
}